{
  "gene": "UniProtKB:Q9H0I9",
  "term_id": "GO:0030976",
  "term_label": "thiamine pyrophosphate binding",
  "gene_symbol": "TKTL2",
  "gene_name": "Transketolase-like protein 2"
}